pyrimidine nucleoside catabolic process [GO:0046135] (biological process) Subtypes: pyrimidine deoxyribonucleoside catabolic process [GO:0046127], pyrimidine ribonucleoside catabolic process [GO:0046133], blasticidin S catabolic process [GO:1905265] Definition: The chemical reactions and pathways resulting in the breakdown of one of a family of organic molecules consisting of a pyrimidine base covalently bonded to a sugar ribose (a ribonucleoside) or deoxyribose (a deoxyribonucleoside). Sources: GOC:ai Relationships: is a type of pyrimidine nucleoside metabolic process [GO:0006213]; is a type of nucleoside catabolic process [GO:0009164]; is a type of pyrimidine-containing compound catabolic process [GO:0072529] Also known as: pyrimidine nucleoside breakdown, pyrimidine nucleoside catabolism, pyrimidine nucleoside degradation